L-glutamate catabolic process via 2-hydroxyglutarate [GO:0019552] (biological process) Definition: The anaerobic chemical reactions and pathways resulting in the breakdown of L-glutamate, via the intermediate 2-hydroxyglutarate, yielding energy in the form of ATP. Sources: MetaCyc:P162-PWY Relationships: is a type of GO:0006083; is a type of anaerobic L-glutamate catabolic process [GO:0019670]; is a type of L-glutamate catabolic process to butyrate [GO:0033508] Also known as: glutamate fermentation via 2-hydroxyglutarate